{
  "gene_symbol": "IFT57",
  "term_label": "intraciliary transport",
  "gene": "UniProtKB:Q9NWB7",
  "term_id": "GO:0042073",
  "gene_name": "Intraflagellar transport protein 57 homolog"
}